CAU codon-amino acid adaptor activity [GO:0033425] (molecular function) Sources: GOC:mah Note: Note that in the standard genetic code, CAT codes for histidine. Definition: A triplet codon-amino acid adaptor activity that recognizes a CAU codon. Relationships: is_a triplet codon-amino acid adaptor activity [GO:0030533] Also known as: CAT codon-amino acid adaptor activity, histidine tRNA